{
  "term_id": "UNKNOWN:0001",
  "gene_name": "Stomatin-like protein 2, mitochondrial",
  "gene": "UniProtKB:Q9UJZ1",
  "term_label": "Unknown molecular function",
  "gene_symbol": "STOML2"
}